{
  "term_label": "cell surface",
  "gene_name": "Pancreatic secretory granule membrane major glycoprotein GP2",
  "gene": "UniProtKB:P55259",
  "gene_symbol": "GP2",
  "term_id": "GO:0009986"
}